chemokine (C-C motif) ligand 20 production [GO:0036392] (biological process) Also known as: C-C motif chemokine 20 production, CCL-20 production, CCL20 production Regulation: regulated by regulation of chemokine (C-C motif) ligand 20 production [GO:1903884]; negatively regulated by negative regulation of chemokine (C-C motif) ligand 20 production [GO:1903885]; positively regulated by positive regulation of chemokine (C-C motif) ligand 20 production [GO:1903886] Sources: GOC:jc Definition: The appearance of chemokine (C-C motif) ligand 20 (CCL20) due to biosynthesis or secretion following a cellular stimulus, resulting in an increase in its intracellular or extracellular levels. Relationships: is a type of chemokine production [GO:0032602]